regulation of tube diameter [GO:0035296] (biological process) Definition: Any process that modulates the diameter of a tube. Sources: GOC:bf Relationships: is a type of regulation of tube size [GO:0035150] Subtypes: GO:0035158, regulation of Malpighian tubule diameter [GO:0035297], blood vessel diameter maintenance [GO:0097746]